negative regulation of granulosa cell proliferation [GO:1904196] (BP) Also known as: down regulation of granulosa cell proliferation, down-regulation of granulosa cell proliferation, downregulation of granulosa cell proliferation, inhibition of granulosa cell proliferation Relationships: is_a negative regulation of epithelial cell proliferation [GO:0050680]; is a type of regulation of granulosa cell proliferation [GO:1904195]; negatively regulates granulosa cell proliferation [GO:1990739] Definition: Any process that stops, prevents or reduces the frequency, rate or extent of granulosa cell proliferation. References: PMID:22383759 Sources: GOC:TermGenie, GO_REF:0000058